{
  "term_id": "GO:0006357",
  "term_label": "regulation of transcription by RNA polymerase II",
  "gene_name": "Homeobox protein Nkx-2.2",
  "gene": "UniProtKB:O95096",
  "gene_symbol": "NKX2-2"
}